{
  "term_label": "external side of plasma membrane",
  "gene_symbol": "BTNL2",
  "gene_name": "Butyrophilin-like protein 2",
  "term_id": "GO:0009897",
  "gene": "UniProtKB:Q9UIR0"
}